positive regulation of gastrulation [GO:2000543] (BP) Definition: Any process that activates or increases the frequency, rate or extent of gastrulation. Sources: GOC:obol Relationships: is a type of regulation of gastrulation [GO:0010470]; is a type of GO:0040019; positively regulates gastrulation [GO:0007369]